{
  "gene": "UniProtKB:Q9UHF3",
  "term_label": "Unknown cellular component",
  "term_id": "UNKNOWN:0003",
  "gene_name": "Putative N-acetyltransferase 8B",
  "gene_symbol": "NAT8B"
}